sorbitol biosynthetic process [GO:0006061] (BP) Relationships: is_a sorbitol metabolic process [GO:0006060]; is a type of GO:0019406 Sources: ISBN:0198506732 Also known as: sorbitol anabolism, sorbitol biosynthesis, sorbitol formation, sorbitol synthesis Definition: The chemical reactions and pathways resulting in the formation of sorbitol (D-glucitol), one of the ten stereoisomeric hexitols. It can be derived from glucose by reduction of the aldehyde group.